{
  "gene_symbol": "N4BP2L1",
  "gene_name": "NEDD4-binding protein 2-like 1",
  "term_label": "Unknown cellular component",
  "gene": "UniProtKB:Q5TBK1",
  "term_id": "UNKNOWN:0003"
}